{
  "term_id": "GO:0006355",
  "gene_name": "Host cell factor 2",
  "term_label": "regulation of DNA-templated transcription",
  "gene": "UniProtKB:Q9Y5Z7",
  "gene_symbol": "HCFC2"
}